negative regulation of sarcomere organization [GO:0060299] (biological process) Sources: GOC:BHF, GOC:dph, GOC:tb Relationships: is a type of GO:0010721; is_a GO:0051494; is a type of GO:0060297; is a type of negative regulation of organelle assembly [GO:1902116]; is a type of GO:1902904; negatively regulates sarcomere organization [GO:0045214] Definition: Any process that decreases the rate, frequency or extent of myofibril assembly by organization of muscle actomyosin into sarcomeres. The sarcomere is the repeating unit of a myofibril in a muscle cell, composed of an array of overlapping thick and thin filaments between two adjacent Z discs. Also known as: negative regulation of sarcomere organisation